{
  "gene": "UniProtKB:Q9UKL0",
  "gene_name": "REST corepressor 1",
  "gene_symbol": "RCOR1",
  "term_label": "negative regulation of DNA-templated transcription",
  "term_id": "GO:0045892"
}